{
  "term_label": "N-acetylglucosamine-6-phosphate deacetylase activity",
  "term_id": "GO:0008448",
  "gene_name": "N-acetylglucosamine-6-phosphate deacetylase",
  "gene_symbol": "AMDHD2",
  "gene": "UniProtKB:Q9Y303"
}